{
  "gene_name": "SAC3 domain-containing protein 1",
  "term_label": "spindle assembly",
  "term_id": "GO:0051225",
  "gene": "UniProtKB:A6NKF1",
  "gene_symbol": "SAC3D1"
}